{
  "term_label": "immune response",
  "gene_symbol": "CEACAM21",
  "gene_name": "Carcinoembryonic antigen-related cell adhesion molecule 21",
  "gene": "UniProtKB:Q3KPI0",
  "term_id": "GO:0006955"
}